{
  "gene": "UniProtKB:P62750",
  "term_label": "cytosolic large ribosomal subunit",
  "gene_name": "Large ribosomal subunit protein uL23",
  "gene_symbol": "RPL23A",
  "term_id": "GO:0022625"
}